{
  "term_label": "Unknown cellular component",
  "gene": "UniProtKB:P0C5K6",
  "gene_symbol": "VENTXP1",
  "gene_name": "Putative tumor antigen NA88-A",
  "term_id": "UNKNOWN:0003"
}